{
  "gene_symbol": "CUL5",
  "term_label": "protein ubiquitination",
  "term_id": "GO:0016567",
  "gene": "UniProtKB:Q93034",
  "gene_name": "Cullin-5"
}